{
  "gene": "UniProtKB:Q6NX45",
  "term_label": "regulation of transcription by RNA polymerase II",
  "gene_name": "Zinc finger protein 774",
  "gene_symbol": "ZNF774",
  "term_id": "GO:0006357"
}